SH2 domain binding [GO:0042169] (molecular function) Definition: Binding to a SH2 domain (Src homology 2) of a protein, a protein domain of about 100 amino-acid residues and belonging to the alpha + beta domain class. Relationships: is a type of protein domain specific binding [GO:0019904] Sources: GOC:go_curators, Pfam:PF00017